citrate CoA-transferase activity [GO:0008814] (molecular function) Also known as: acetyl-CoA:citrate CoA-transferase activity Definition: Catalysis of the reaction: acetyl-CoA + citrate = acetate + (3S)-citryl-CoA. Sources: EC:2.8.3.10 Relationships: is a type of CoA-transferase activity [GO:0008410]